{
  "gene_name": "TBC1 domain family member 2A",
  "gene": "UniProtKB:Q9BYX2",
  "term_id": "GO:0005737",
  "term_label": "cytoplasm",
  "gene_symbol": "TBC1D2"
}